{
  "gene": "UniProtKB:Q6ZMR3",
  "gene_symbol": "LDHAL6A",
  "gene_name": "L-lactate dehydrogenase A-like 6A",
  "term_id": "GO:0006089",
  "term_label": "lactate metabolic process"
}